{
  "gene_name": "Protein ITPRID1",
  "term_label": "Unknown biological process",
  "gene": "UniProtKB:Q6ZRS4",
  "term_id": "UNKNOWN:0002",
  "gene_symbol": "ITPRID1"
}